{
  "term_label": "Unknown molecular function",
  "gene_symbol": "SCRN1",
  "term_id": "UNKNOWN:0001",
  "gene": "UniProtKB:Q12765",
  "gene_name": "Secernin-1"
}